telomere maintenance via base-excision repair [GO:0097698] (biological process) References: PMID:24703901 Sources: GOC:BHF, GOC:BHF_telomere, GOC:jbu Relationships: is a type of GO:0006284; is a type of telomere maintenance in response to DNA damage [GO:0043247] Definition: A telomere maintenance process that occurs by base-excision repair of telomeric DNA in response to DNA damage. Telomeric sequences are particularly susceptible to oxidative DNA damage, due to their G-rich nature.